{
  "term_label": "cyclin-dependent protein serine/threonine kinase regulator activity",
  "gene_name": "Cyclin-Q",
  "gene": "UniProtKB:Q8N1B3",
  "term_id": "GO:0016538",
  "gene_symbol": "CCNQ"
}